glycogen catabolic process via dextrin [GO:0160251] (biological process) Sources: MetaCyc:PWY-5941 Relationships: is a type of glycogen catabolic process [GO:0005980] Definition: The chemical reactions and pathways resulting in the breakdown of glycogen, a polydisperse, highly branched glucan composed of chains of D-glucose residues, occurring through dextrin derivative intermediates.